{
  "term_id": "GO:0004064",
  "gene": "UniProtKB:Q9HDC9",
  "term_label": "arylesterase activity",
  "gene_name": "Adipocyte plasma membrane-associated protein",
  "gene_symbol": "APMAP"
}